{
  "gene_symbol": "VAMP3",
  "term_label": "SNARE complex",
  "gene": "UniProtKB:Q15836",
  "term_id": "GO:0031201",
  "gene_name": "Vesicle-associated membrane protein 3"
}